{
  "gene_symbol": "CA5B",
  "gene_name": "Carbonic anhydrase 5B, mitochondrial",
  "gene": "UniProtKB:Q9Y2D0",
  "term_label": "mitochondrion",
  "term_id": "GO:0005739"
}